{
  "term_id": "GO:0097250",
  "gene_symbol": "HIGD2B",
  "term_label": "mitochondrial respirasome assembly",
  "gene_name": "Putative HIG1 domain family member 2B",
  "gene": "UniProtKB:Q4VC39"
}